{
  "gene_symbol": "MAGEA9",
  "gene_name": "Melanoma-associated antigen 9",
  "term_label": "histone deacetylase binding",
  "term_id": "GO:0042826",
  "gene": "UniProtKB:P43362"
}